static microtubule bundle [GO:0099070] (CC) References: PMID:26124291 Sources: GOC:vw Definition: A microtubule bundle that has a constant length, and in which microtubule sliding does not take place. Note: In fission yeast, quiescent cells contain only static microtubule bundles. Also known as: Q-MT bundle, quiescent cell MT bundle, quiescent cell microtubule bundle Relationships: is a type of microtubule bundle [GO:0097427]